{
  "term_id": "UNKNOWN:0003",
  "gene": "UniProtKB:B0L3A2",
  "term_label": "Unknown cellular component",
  "gene_name": "Dual endothelin-1_angiotensin II receptor",
  "gene_symbol": "FBXW7-AS1"
}